3'-deoxyribose phosphate lyase activity [GO:0106334] (MF) Relationships: is a type of lyase activity [GO:0016829]; is a type of catalytic activity, acting on DNA [GO:0140097] Definition: Catalysis of the conversion of a 3'-deoxyribose phosphate in DNA to a 3'-phosphate. References: PMID:21276450, PMID:22084197, PMID:22375014 Sources: GOC:mah, RHEA:65764 Also known as: 3'-dRP lyase, 3'-dRP lyase activity